neuron projection branch point [GO:0061845] (CC) Relationships: is a type of GO:0110165; is part of neuron projection [GO:0043005] Subtypes: dendritic branch point [GO:1990033] References: PMID:25586189 Definition: The location where a secondary projection arises from a neuron projection.